{
  "term_label": "Unknown cellular component",
  "term_id": "UNKNOWN:0003",
  "gene_symbol": "OR5M8",
  "gene_name": "Olfactory receptor 5M8",
  "gene": "UniProtKB:Q8NGP6"
}